{
  "gene": "UniProtKB:Q6IQ23",
  "gene_symbol": "PLEKHA7",
  "term_id": "GO:0090136",
  "term_label": "epithelial cell-cell adhesion",
  "gene_name": "Pleckstrin homology domain-containing family A member 7"
}